{
  "term_label": "regulation of mitotic cell cycle",
  "gene_name": "Serine_threonine-protein kinase pim-3",
  "term_id": "GO:0007346",
  "gene": "UniProtKB:Q86V86",
  "gene_symbol": "PIM3"
}